viral occlusion body [GO:0039679] (cellular component) Sources: UniProtKB-KW:KW-0842, VZ:1949 Relationships: is a type of pathogen-containing vacuole [GO:0140220] Definition: A crystalline protein matrix surrounding the nucleocapsids of some insect viruses after their release in the environment. Produced in the host cell, the occlusion body protects the infectious virion after death of the host.